retinyl-palmitate esterase activity [GO:0050253] (molecular function) Relationships: is a type of carboxylic ester hydrolase activity [GO:0052689]; BFO_0000050 retinol metabolic process [GO:0042572] Also known as: retinyl ester hydrolase activity, retinyl palmitate hydrolase activity, retinyl palmitate hydrolyase activity, retinyl-palmitate palmitohydrolase activity Subtypes: GO:0047376, all-trans-retinyl-palmitate hydrolase, 11-cis retinol forming activity [GO:0052884] Sources: RHEA:21508 Definition: Catalysis of the reaction: retinyl palmitate + H2O = retinol + palmitate + H+.